{
  "gene_name": "Scavenger receptor class B member 1",
  "gene_symbol": "SCARB1",
  "term_label": "cholesterol efflux",
  "term_id": "GO:0033344",
  "gene": "UniProtKB:Q8WTV0"
}